{
  "term_label": "Unknown cellular component",
  "gene_name": "Putative uncharacterized protein FAM30A",
  "gene_symbol": "FAM30A",
  "gene": "UniProtKB:Q9NZY2",
  "term_id": "UNKNOWN:0003"
}